methylmercury biosynthetic process [GO:0042192] (BP) Note: Note that there is no unequivocal evidence supporting a specific physiological role for the reaction leading to the synthesis of methylmercury. It may be a defense molecule, or serve to detoxify mercury. Once the physiological role is understood, this term will likely be obsoleted. Also known as: methylmercury anabolism, methylmercury biosynthesis, methylmercury formation, methylmercury synthesis Definition: The chemical reactions and pathways resulting in the formation of methylmercury (MeHg+), a highly toxic organometal. References: PMID:23393089, PMID:38407657 Sources: GOC:ai Relationships: is a type of biosynthetic process [GO:0009058]; is a type of organometal metabolic process [GO:0018942]